autophagosome-lysosome fusion [GO:0061909] (biological process) Regulation: positively regulated by GO:0160177 Also known as: autophagosome fusion, autophagosome-vacuole fusion Relationships: is a type of GO:0006906; is part of macroautophagy [GO:0016236] Definition: The process in which autophagosomes, double-membraned vesicles containing cytoplasmic material, fuse with a vacuole (yeast) or lysosome (e.g. mammals and insects). In the case of yeast, inner membrane-bounded structures (autophagic bodies) appear in the vacuole. Fusion provides an acidic environment and digestive function to the interior of the autophagosome. References: PMID:28077293